{
  "term_id": "GO:0003729",
  "gene_symbol": "LSM14A",
  "gene": "UniProtKB:Q8ND56",
  "term_label": "mRNA binding",
  "gene_name": "Protein LSM14 homolog A"
}